{
  "term_label": "cytosol",
  "gene": "UniProtKB:Q9UMW8",
  "gene_symbol": "USP18",
  "gene_name": "Ubl carboxyl-terminal hydrolase 18",
  "term_id": "GO:0005829"
}